brassinosteroid sulfotransferase activity [GO:0080118] (molecular function) Definition: Catalysis of the reaction: a brassinosteroid + 3'-phosphoadenosine-5'-phosphosulfate = sulfated brassinosteroid + adenosine-3',5'-diphosphate. This reaction is the transfer of a sulfate group to the hydroxyl group of a brassinosteroid acceptor, producing the sulfated brassinosteroid derivative. References: PMID:10409637, PMID:17039368 Relationships: is a type of sulfotransferase activity [GO:0008146]